{
  "gene_name": "Serine protease HTRA4",
  "term_label": "programmed cell death",
  "gene_symbol": "HTRA4",
  "term_id": "GO:0012501",
  "gene": "UniProtKB:P83105"
}